{
  "gene_name": "Transcription factor JunD",
  "term_id": "GO:0005667",
  "gene_symbol": "JUND",
  "term_label": "transcription regulator complex",
  "gene": "UniProtKB:P17535"
}